{
  "term_label": "protein localization to kinetochore",
  "gene_name": "Protein zwilch homolog",
  "gene_symbol": "ZWILCH",
  "gene": "UniProtKB:Q9H900",
  "term_id": "GO:0034501"
}